phenanthrene-9,10-epoxide hydrolase activity [GO:0019119] (molecular function) Relationships: is a type of phenanthrene-epoxide hydrolase activity [GO:0019118] Sources: GOC:mah, UM-BBD_reactionID:r0496, UM-BBD_reactionID:r0560 Definition: Catalysis of the reaction: phenanthrene-9,10-oxide + H2O = trans-9,10-dihydrodiolphenanthrene.